{
  "gene_symbol": "LOC122455340",
  "gene": "UniProtKB:A0A1B0GVY2",
  "term_label": "Unknown molecular function",
  "gene_name": "Uncharacterized protein",
  "term_id": "UNKNOWN:0001"
}